{
  "gene": "UniProtKB:A6NKT7",
  "term_label": "NLS-bearing protein import into nucleus",
  "gene_symbol": "RGPD3",
  "term_id": "GO:0006607",
  "gene_name": "RanBP2-like and GRIP domain-containing protein 3"
}